CSK-GAP-A.p62 complex [GO:0070214] (cellular component) References: PMID:7544435 Definition: A protein complex that contains the protein-tyrosine kinase CSK and the GTPase-activating protein (GAP)-associated p62 (GAP-A.p62); may mediate translocation of proteins, including GAP and CSK, to membrane or cytoskeletal regions upon c-Src activation. Note: Note that the gene/protein name 'APC' should not be confused with the abbreviation for 'anaphase promoting complex'. Relationships: is a type of intracellular protein-containing complex [GO:0140535]; is a type of catalytic complex [GO:1902494]; is part of cell leading edge [GO:0031252]